{
  "gene_name": "Platelet-activating factor acetylhydrolase IB subunit beta",
  "term_id": "GO:0008090",
  "gene": "UniProtKB:P43034",
  "term_label": "retrograde axonal transport",
  "gene_symbol": "PAFAH1B1"
}